{
  "gene_symbol": "MED13",
  "gene_name": "Mediator of RNA polymerase II transcription subunit 13",
  "gene": "UniProtKB:Q9UHV7",
  "term_id": "GO:0045944",
  "term_label": "positive regulation of transcription by RNA polymerase II"
}